{
  "gene_name": "Protein ripply3",
  "gene_symbol": "RIPPLY3",
  "term_id": "GO:0000122",
  "term_label": "negative regulation of transcription by RNA polymerase II",
  "gene": "UniProtKB:P57055"
}